{
  "term_id": "GO:0000122",
  "gene_name": "Melanoma-associated antigen H1",
  "term_label": "negative regulation of transcription by RNA polymerase II",
  "gene_symbol": "MAGEH1",
  "gene": "UniProtKB:Q9H213"
}